{
  "gene_name": "Ankyrin repeat domain-containing protein 27",
  "term_id": "GO:0005770",
  "gene_symbol": "ANKRD27",
  "term_label": "late endosome",
  "gene": "UniProtKB:Q96NW4"
}